{
  "gene_symbol": "MIR1-1HG",
  "term_label": "Unknown cellular component",
  "gene": "UniProtKB:Q9H1L0",
  "term_id": "UNKNOWN:0003",
  "gene_name": "Uncharacterized protein MIR1-1HG"
}